{
  "gene": "UniProtKB:B7U540",
  "gene_name": "Inward rectifier potassium channel 18",
  "gene_symbol": "KCNJ18",
  "term_id": "UNKNOWN:0001",
  "term_label": "Unknown molecular function"
}